{
  "gene_symbol": "ZBTB12",
  "term_label": "negative regulation of transcription by RNA polymerase II",
  "gene": "UniProtKB:Q9Y330",
  "term_id": "GO:0000122",
  "gene_name": "Zinc finger and BTB domain-containing protein 12"
}